glycoside transport [GO:1901656] (biological process) Sources: GOC:TermGenie, GOC:pr Relationships: is a type of GO:1901264 Subtypes: methylgalactoside transport [GO:0015765], GO:0015779, glucoside transport [GO:0042946], daunorubicin transport [GO:0043215], glucosylglycerol transmembrane transport [GO:0051475], phosphoenolpyruvate-dependent mannosylglycerate phosphotransferase system [GO:0051476], doxorubicin transport [GO:1900753] Definition: The directed movement of a glycoside into, out of or within a cell, or between cells, by means of some agent such as a transporter or pore.